{
  "gene_symbol": "DDX52",
  "gene_name": "Probable ATP-dependent RNA helicase DDX52",
  "gene": "UniProtKB:Q9Y2R4",
  "term_label": "maturation of SSU-rRNA",
  "term_id": "GO:0030490"
}